{
  "term_label": "small GTPase binding",
  "gene_symbol": "RABGAP1",
  "gene_name": "Rab GTPase-activating protein 1",
  "term_id": "GO:0031267",
  "gene": "UniProtKB:Q9Y3P9"
}